{
  "gene_symbol": "UBE2F",
  "term_id": "GO:0005829",
  "term_label": "cytosol",
  "gene": "UniProtKB:Q969M7",
  "gene_name": "NEDD8-conjugating enzyme UBE2F"
}